{
  "term_label": "positive regulation of ERK1 and ERK2 cascade",
  "gene": "UniProtKB:P46109",
  "term_id": "GO:0070374",
  "gene_name": "Crk-like protein",
  "gene_symbol": "CRKL"
}